{
  "gene": "UniProtKB:Q9H165",
  "gene_name": "B-cell lymphoma_leukemia 11A",
  "term_id": "GO:0006357",
  "term_label": "regulation of transcription by RNA polymerase II",
  "gene_symbol": "BCL11A"
}